{
  "gene": "UniProtKB:Q6ZS81",
  "term_id": "UNKNOWN:0001",
  "gene_symbol": "WDFY4",
  "gene_name": "WD repeat- and FYVE domain-containing protein 4",
  "term_label": "Unknown molecular function"
}